{
  "term_label": "adenylate cyclase inhibitor activity",
  "gene_name": "Adhesion G-protein coupled receptor V1",
  "term_id": "GO:0010855",
  "gene": "UniProtKB:Q8WXG9",
  "gene_symbol": "ADGRV1"
}